{
  "gene_name": "Sideroflexin-3",
  "gene": "UniProtKB:Q9BWM7",
  "gene_symbol": "SFXN3",
  "term_id": "GO:0140300",
  "term_label": "serine import into mitochondrion"
}